negative regulation of interferon-alpha production [GO:0032687] (biological process) Also known as: down regulation of interferon-alpha production, down-regulation of interferon-alpha production, downregulation of interferon-alpha production, inhibition of interferon-alpha production, negative regulation of interferon-alpha biosynthetic process, negative regulation of interferon-alpha secretion Definition: Any process that stops, prevents, or reduces the frequency, rate, or extent of interferon-alpha production. Relationships: is a type of negative regulation of type I interferon production [GO:0032480]; is a type of regulation of interferon-alpha production [GO:0032647]; negatively regulates interferon-alpha production [GO:0032607] References: PMID:15546383 Sources: GOC:mah